{
  "gene_name": "Single-minded homolog 2",
  "gene_symbol": "SIM2",
  "term_label": "nucleus",
  "term_id": "GO:0005634",
  "gene": "UniProtKB:Q14190"
}